{
  "gene_symbol": "ASB4",
  "term_id": "UNKNOWN:0002",
  "term_label": "Unknown biological process",
  "gene_name": "Ankyrin repeat and SOCS box protein 4",
  "gene": "UniProtKB:Q9Y574"
}